positive regulation of kinin cascade [GO:0002258] (biological process) Also known as: up regulation of kinin cascade, up-regulation of kinin cascade, upregulation of kinin cascade, activation of kinin cascade, stimulation of kinin cascade Relationships: is a type of regulation of kinin cascade [GO:0002256]; is a type of positive regulation of acute inflammatory response [GO:0002675]; is a type of GO:2000259; positively regulates GO:0002254 Sources: GOC:jal Definition: Any process that activates or increases the frequency, rate, or extent of the kinin cascade. Subtypes: positive regulation of tissue kallikrein-kinin cascade [GO:0002547], positive regulation of plasma kallikrein-kinin cascade [GO:0002550]